{
  "term_label": "plasma membrane",
  "gene": "UniProtKB:P09497",
  "gene_symbol": "CLTB",
  "term_id": "GO:0005886",
  "gene_name": "Clathrin light chain B"
}